negative regulation of glial cell proliferation [GO:0060253] (biological process) Definition: Any process that stops or decreases the rate or extent of glial cell proliferation. Subtypes: GO:0010626 Relationships: is a type of negative regulation of cell population proliferation [GO:0008285]; is a type of negative regulation of gliogenesis [GO:0014014]; is a type of regulation of glial cell proliferation [GO:0060251]; negatively regulates glial cell proliferation [GO:0014009] Sources: GOC:dph, GOC:sl, GOC:tb